{
  "term_label": "nucleus",
  "gene": "UniProtKB:Q96RK0",
  "term_id": "GO:0005634",
  "gene_name": "Protein capicua homolog",
  "gene_symbol": "CIC"
}